{
  "gene_symbol": "APOBEC3F",
  "term_label": "nucleus",
  "gene_name": "DNA dC-dU-editing enzyme APOBEC-3F",
  "term_id": "GO:0005634",
  "gene": "UniProtKB:Q8IUX4"
}